negative regulation of spermatid nuclear differentiation [GO:0045701] (biological process) Also known as: down regulation of spermatid nuclear differentiation, down-regulation of spermatid nuclear differentiation, downregulation of spermatid nuclear differentiation, inhibition of spermatid nuclear differentiation Sources: GOC:go_curators Relationships: is a type of negative regulation of organelle organization [GO:0010639]; is a type of GO:0045596; is a type of GO:0045700; is a type of GO:0051241; is a type of negative regulation of reproductive process [GO:2000242]; negatively regulates spermatid nucleus differentiation [GO:0007289] Definition: Any process that stops, prevents, or reduces the frequency, rate or extent of spermatid nuclear differentiation.